{
  "term_label": "ubiquitin-like ligase-substrate adaptor activity",
  "gene_symbol": "KLHL40",
  "term_id": "GO:1990756",
  "gene": "UniProtKB:Q2TBA0",
  "gene_name": "Kelch-like protein 40"
}